{
  "gene_name": "Junctional adhesion molecule B",
  "term_label": "protein complex involved in cell adhesion",
  "gene_symbol": "JAM2",
  "term_id": "GO:0098636",
  "gene": "UniProtKB:P57087"
}